negative regulation of angiogenesis [GO:0016525] (biological process) Relationships: is a type of regulation of angiogenesis [GO:0045765]; is a type of negative regulation of blood vessel morphogenesis [GO:2000181]; negatively regulates GO:0001525 Definition: Any process that stops, prevents, or reduces the frequency, rate or extent of angiogenesis. Sources: GOC:go_curators Subtypes: negative regulation of vascular wound healing [GO:0061044], GO:1903671, negative regulation of blood vessel branching [GO:1905554] Also known as: down regulation of angiogenesis, down-regulation of angiogenesis, downregulation of angiogenesis, inhibition of angiogenesis